{
  "gene_name": "HLA class II histocompatibility antigen, DO beta chain",
  "gene_symbol": "HLA-DOB",
  "term_label": "positive regulation of immune response",
  "gene": "UniProtKB:P13765",
  "term_id": "GO:0050778"
}